{
  "gene": "UniProtKB:Q92772",
  "term_id": "UNKNOWN:0002",
  "gene_name": "Cyclin-dependent kinase-like 2",
  "gene_symbol": "CDKL2",
  "term_label": "Unknown biological process"
}